neuron migration involved in amphid sensory organ dendrite retrograde extension [GO:0003397] (biological process) Relationships: is a type of GO:0003395; is part of amphid sensory organ dendrite retrograde extension [GO:0003391] Definition: The directed, self-propelled movement of a neuron that contributes to the process of retrograde extension of a dendrite of a neuron in the amphid sensory organ. Sources: GOC:ascb_2009, GOC:dph, GOC:tb